{
  "gene": "UniProtKB:Q9BTY7",
  "gene_symbol": "HGH1",
  "term_label": "Unknown cellular component",
  "gene_name": "Protein HGH1 homolog",
  "term_id": "UNKNOWN:0003"
}